pigment cell precursor differentiation [GO:0048824] (biological process) Relationships: is a type of GO:0030154 Definition: The process in which a relatively unspecialized cell acquires specialized features of a pigment cell precursor. Also known as: chromatophore precursor differentiation References: PMID:16499899 Sources: GOC:dgh